{
  "term_id": "GO:0050877",
  "term_label": "nervous system process",
  "gene": "UniProtKB:P51825",
  "gene_symbol": "AFF1",
  "gene_name": "AF4_FMR2 family member 1"
}